{
  "gene_name": "Dihydroorotate dehydrogenase (quinone), mitochondrial",
  "gene_symbol": "DHODH",
  "term_id": "GO:0009220",
  "gene": "UniProtKB:Q02127",
  "term_label": "pyrimidine ribonucleotide biosynthetic process"
}